{
  "gene_name": "ADP-ribosyl cyclase_cyclic ADP-ribose hydrolase 1",
  "gene": "UniProtKB:P28907",
  "term_id": "GO:0016849",
  "gene_symbol": "CD38",
  "term_label": "phosphorus-oxygen lyase activity"
}